bundle of His cell action potential [GO:0086043] (biological process) Relationships: is a type of cardiac muscle cell action potential [GO:0086001]; is part of bundle of His cell to Purkinje myocyte signaling [GO:0086028] Regulation: RO_0002211 by regulation of bundle of His cell action potential [GO:0098905] Definition: An action potential that occurs in a bundle of His cell. Sources: GOC:BHF, GOC:mtg_cardiac_conduct_nov11 Also known as: bundle of His cardiac muscle cell action potential